{
  "gene_symbol": "A0A494C0I6",
  "term_label": "Unknown biological process",
  "gene": "UniProtKB:A0A494C0I6",
  "term_id": "UNKNOWN:0002",
  "gene_name": "Uncharacterized protein"
}